{
  "gene_name": "Ryanodine receptor 1",
  "gene": "UniProtKB:P21817",
  "term_label": "striated muscle contraction",
  "gene_symbol": "RYR1",
  "term_id": "GO:0006941"
}